{
  "gene_name": "LIM_homeobox protein Lhx8",
  "term_id": "GO:0030182",
  "gene_symbol": "LHX8",
  "term_label": "neuron differentiation",
  "gene": "UniProtKB:Q68G74"
}